{
  "term_label": "sister chromatid cohesion",
  "term_id": "GO:0007062",
  "gene": "UniProtKB:Q14683",
  "gene_name": "Structural maintenance of chromosomes protein 1A",
  "gene_symbol": "SMC1A"
}